{
  "term_label": "GTP binding",
  "gene_symbol": "ARL5B",
  "gene_name": "ADP-ribosylation factor-like protein 5B",
  "gene": "UniProtKB:Q96KC2",
  "term_id": "GO:0005525"
}